{
  "gene_name": "Soluble scavenger receptor cysteine-rich domain-containing protein SSC5D",
  "gene": "UniProtKB:A1L4H1",
  "term_label": "defense response",
  "term_id": "GO:0006952",
  "gene_symbol": "SSC5D"
}